{
  "gene": "UniProtKB:Q92625",
  "gene_name": "Ankyrin repeat and SAM domain-containing protein 1A",
  "term_label": "ephrin receptor binding",
  "gene_symbol": "ANKS1A",
  "term_id": "GO:0046875"
}